rhombomere 6 formation [GO:0021669] (biological process) Definition: The process that gives rise to rhombomere 6. This process pertains to the initial formation of a structure from unspecified parts. Rhombomeres are transverse segments of the developing rhombencephalon. Rhombomeres are lineage restricted, express different genes from one another, and adopt different developmental fates. Rhombomeres are numbered in anterior to posterior order. Sources: GOC:cls, GOC:curators, GOC:dgh, GOC:dph, GOC:jid Relationships: is a type of GO:0021594; is part of rhombomere 6 morphogenesis [GO:0021667]